carbon-nitrogen ligase activity on lipid II [GO:0140282] (molecular function) Relationships: is a type of carbon-nitrogen ligase activity, with glutamine as amido-N-donor [GO:0016884] Also known as: L-glutamate--lipid II transaminase activity, undecaprenyldiphospho-N-acetyl-(N-acetylglucosaminyl)muramoyl pentapeptide amidotransferase (glutamine-hydrolyzing) activity References: PMID:22291598, PMID:30093673, PMID:30154570 Sources: RHEA:57928 Definition: Catalysis of the reaction: L-glutamine + lipid II + ATP + H2O = L-glutamate + beta-D-GlcNAc(1->4)-Mur2Ac(oyl-L-Ala-D-isoGln-L-Lys-D-Ala-D-Ala)-diphospho-di-trans,octa-cis-undecaprenol + ADP + phosphate.